rosmarinate synthase activity [GO:0050266] (molecular function) Also known as: 4-coumaroyl-CoA:4-hydroxyphenyllactic acid 4-coumaroyl transferase activity, caffeoyl-CoA:3-(3,4-dihydroxyphenyl)lactate 2'-O-caffeoyl-transferase activity, caffeoyl-coenzyme A:3,4-dihydroxyphenyllactic acid caffeoyltransferase activity, rosmarinic acid synthase activity Definition: Catalysis of the reaction: caffeoyl-CoA + 3-(3,4-dihydroxyphenyl)lactate = CoA + rosmarinate. Sources: EC:2.3.1.140 Relationships: is a type of acyltransferase activity, transferring groups other than amino-acyl groups [GO:0016747]